polytene chromosome ectopic fiber [GO:0005706] (cellular component) Sources: GOC:bf, ISBN:0120649012 Relationships: is_a cellular anatomical structure [GO:0110165]; BFO_0000050 polytene chromosome [GO:0005700] Also known as: polytene chromosome ectopic fibre Definition: A thread-like connection joining two regions of ectopically paired polytene chromosomes.